{
  "term_label": "histone binding",
  "gene": "UniProtKB:P33552",
  "term_id": "GO:0042393",
  "gene_name": "Cyclin-dependent kinases regulatory subunit 2",
  "gene_symbol": "CKS2"
}